{
  "gene_symbol": "TMEM276",
  "gene": "UniProtKB:P0DTL5",
  "term_id": "UNKNOWN:0001",
  "gene_name": "Transmembrane protein 276",
  "term_label": "Unknown molecular function"
}